{
  "gene_symbol": "OLIG1",
  "gene_name": "Oligodendrocyte transcription factor 1",
  "term_label": "axon development",
  "term_id": "GO:0061564",
  "gene": "UniProtKB:Q8TAK6"
}